{
  "gene_name": "Putative protein ZBED10P",
  "gene_symbol": "ZBED10P",
  "term_id": "UNKNOWN:0002",
  "term_label": "Unknown biological process",
  "gene": "UniProtKB:Q96FA7"
}